{
  "gene_symbol": "KLRG1",
  "term_label": "Unknown molecular function",
  "term_id": "UNKNOWN:0001",
  "gene_name": "Killer cell lectin-like receptor subfamily G member 1",
  "gene": "UniProtKB:Q96E93"
}